{
  "term_id": "GO:0005634",
  "gene_name": "5'-3' exoribonuclease 1",
  "gene_symbol": "XRN1",
  "term_label": "nucleus",
  "gene": "UniProtKB:Q8IZH2"
}